{
  "term_id": "GO:0004930",
  "term_label": "G protein-coupled receptor activity",
  "gene": "UniProtKB:Q8N6U8",
  "gene_name": "G-protein coupled receptor 161",
  "gene_symbol": "GPR161"
}